histone H3K56ac reader activity [GO:0140129] (molecular function) Definition: A histone reader that recognizes a histone H3 acetylated at lysine 56. References: PMID:23798425 Note: Comment: Note that the residue position corresponds to the canonical human H3 histone (UniProtKB:P84243); this residue is conserved across all eukaryotes. Residue 1 is the first residue following removal of the initiating Methionine (Met). Note that each histone is encoded by multiple genes, and sequences may vary across different genes within an organism. Relationships: is a type of histone H3 reader activity [GO:0140006]